{
  "term_label": "Unknown molecular function",
  "gene_name": "Golgin subfamily A member 8A",
  "gene_symbol": "GOLGA8A",
  "gene": "UniProtKB:A7E2F4",
  "term_id": "UNKNOWN:0001"
}